{
  "term_label": "regulation of transcription by RNA polymerase II",
  "gene_symbol": "BARX1",
  "term_id": "GO:0006357",
  "gene": "UniProtKB:Q9HBU1",
  "gene_name": "Homeobox protein BarH-like 1"
}